donor selection [GO:0007535] (biological process) Relationships: is a type of developmental process involved in reproduction [GO:0003006]; is a type of cellular developmental process [GO:0048869]; is part of mating type switching [GO:0007533] References: PMID:9928492 Sources: GOC:mah Also known as: donor preference Definition: The process that determines which donor locus a cell uses, in preference to another, in mating type switching. Subtypes: activation of recombination (HML) [GO:0007536], inactivation of recombination (HML) [GO:0007537]